regulation of neural precursor cell proliferation [GO:2000177] (biological process) Sources: GOC:dph, GOC:yaf Subtypes: regulation of cell proliferation in dorsal spinal cord [GO:0021921], regulation of cerebellar granule cell precursor proliferation [GO:0021936], GO:0070445, regulation of neuroblast proliferation [GO:1902692], GO:1904933, negative regulation of neural precursor cell proliferation [GO:2000178], positive regulation of neural precursor cell proliferation [GO:2000179] Relationships: is a type of GO:0042127; regulates neural precursor cell proliferation [GO:0061351] Definition: Any process that modulates the frequency, rate or extent of neural precursor cell proliferation.